{
  "term_label": "Unknown biological process",
  "term_id": "UNKNOWN:0002",
  "gene": "UniProtKB:Q66K14",
  "gene_name": "TBC1 domain family member 9B",
  "gene_symbol": "TBC1D9B"
}